{
  "gene_name": "Claudin-11",
  "term_id": "GO:0007155",
  "gene": "UniProtKB:O75508",
  "gene_symbol": "CLDN11",
  "term_label": "cell adhesion"
}